{
  "term_label": "Unknown biological process",
  "term_id": "UNKNOWN:0002",
  "gene_name": "Family with sequence similarity 90 member A3, pseudogene",
  "gene_symbol": "FAM90A3P",
  "gene": "UniProtKB:A0A8V8TPE2"
}